2-ethylmalate synthase activity [GO:0050438] (molecular function) Also known as: (R)-2-ethylmalate 2-oxobutanoyl-lyase (CoA-acetylating) activity, 2-ethylmalate-3-hydroxybutanedioate synthase activity, acetyl-CoA:2-oxobutanoate C-acetyltransferase (thioester-hydrolysing, carboxymethyl-forming), propylmalate synthase activity, propylmalic synthase activity Sources: RHEA:23040 Definition: Catalysis of the reaction: 2-oxobutanate + acetyl-CoA + H2O = (R)-2-ethylmalate + CoA + H+. Relationships: is a type of acyltransferase activity, acyl groups converted into alkyl on transfer [GO:0046912]